3-(3-hydroxyphenyl)propionate hydroxylase activity [GO:0008688] (molecular function) Relationships: is a type of oxidoreductase activity, acting on paired donors, with incorporation or reduction of molecular oxygen, NAD(P)H as one donor, and incorporation of one atom of oxygen [GO:0016709] Definition: Catalysis of the reaction: 3-(3-hydroxyphenyl)propionate + NADH + oxygen + H+ = 3-(2,3-dihydroxyphenyl)propionate + NAD+ + H2O. Sources: RHEA:24785